{
  "gene_symbol": "SNX3",
  "gene": "UniProtKB:O60493",
  "term_id": "GO:0031901",
  "gene_name": "Sorting nexin-3",
  "term_label": "early endosome membrane"
}